{
  "gene_name": "Uncharacterized protein C9orf152",
  "term_label": "Unknown molecular function",
  "gene": "UniProtKB:Q5JTZ5",
  "gene_symbol": "C9orf152",
  "term_id": "UNKNOWN:0001"
}